{
  "gene": "UniProtKB:Q9NPG8",
  "gene_name": "Palmitoyltransferase ZDHHC4",
  "term_label": "Golgi apparatus",
  "gene_symbol": "ZDHHC4",
  "term_id": "GO:0005794"
}